cyclosporin A binding [GO:0016018] (molecular function) Also known as: cyclophilin Relationships: is a type of amide binding [GO:0033218] Definition: Binding to cyclosporin A, a cyclic undecapeptide that contains several N-methylated and unusual amino acids. Sources: GOC:mb